pigment granule dispersal [GO:0051876] (biological process) Definition: The directed movement of pigment granules within a cell towards the cell periphery. Sources: GOC:mh Relationships: is a type of establishment of pigment granule localization [GO:0051905]